{
  "gene": "UniProtKB:Q8N6S5",
  "gene_symbol": "ARL6IP6",
  "term_label": "Unknown biological process",
  "gene_name": "ADP-ribosylation factor-like protein 6-interacting protein 6",
  "term_id": "UNKNOWN:0002"
}